all-trans retinoic acid 4-hydrolase activity [GO:0062182] (molecular function) References: PMID:9250660, PMID:9716180 Sources: RHEA:51492 Definition: Catalysis of the reaction: all-trans-retinoate + O2 + reduced [NADPH--hemoprotein reductase] = all-trans-(4S)-hydroxyretinoate + H+ + H2O + oxidized [NADPH--hemoprotein reductase]. Relationships: is_a GO:0008401